galactose uniporter activity [GO:0050782] (molecular function) Sources: GOC:ai, TC:2.A.1.1.6 Relationships: is a type of galactose transmembrane transporter activity [GO:0005354]; is a type of GO:0008516 Definition: Enables the transfer of a solute or solutes from one side of a membrane to the other according to the reaction: galactose (out) = galactose(in). Also known as: galactose, glucose uniporter activity